synaptic target inhibition [GO:0016201] (biological process) Sources: GOC:mah, ISBN:0878932437 Definition: The process in which a neuronal cell in a multicellular organism recognizes chemorepellent signals that inhibit its growth toward the source. Relationships: is a type of negative chemotaxis [GO:0050919]; is part of synaptic target recognition [GO:0008039]